positive regulation of oligodendrocyte progenitor proliferation [GO:0070447] (BP) Definition: Any process that activates or increases the rate or extent of oligodendrocyte progenitor proliferation. Relationships: is a type of positive regulation of gliogenesis [GO:0014015]; is a type of regulation of oligodendrocyte progenitor proliferation [GO:0070445]; is a type of positive regulation of neural precursor cell proliferation [GO:2000179]; positively regulates oligodendrocyte progenitor proliferation [GO:0070444] Also known as: positive regulation of oligodendrocyte precursor proliferation Sources: GOC:mah, GOC:sl